{
  "gene": "UniProtKB:Q96PT4",
  "term_label": "DNA-binding transcription factor activity, RNA polymerase II-specific",
  "gene_symbol": "DUX3",
  "gene_name": "Putative double homeobox protein 3",
  "term_id": "GO:0000981"
}